I-kappaB phosphorylation [GO:0007252] (biological process) References: PMID:21772278, PMID:7594468 Sources: GOC:bf, GOC:jl Regulation: regulated by GO:1903719; negatively regulated by negative regulation of I-kappaB phosphorylation [GO:1903720]; positively regulated by positive regulation of I-kappaB phosphorylation [GO:1903721] Relationships: is_a protein phosphorylation [GO:0006468]; is part of canonical NF-kappaB signal transduction [GO:0007249] Also known as: IKB phosphorylation, IkappaB phosphorylation, inhibitor of NF-kappaB phosphorylation, inhibitor of kappaB phosphorylation Definition: The process of introducing a phosphate group into an inhibitor of kappa B (I-kappaB) protein. Phosphorylation of I-kappaB targets I-kappaB for ubiquitination and proteasomal degradation, thus releasing bound NF-kappaB dimers, which can translocate to the nucleus to bind DNA and regulate transcription.